acetate ester transmembrane transporter activity [GO:1901375] (molecular function) Relationships: is_a transmembrane transporter activity [GO:0022857]; is part of acetate ester transport [GO:1901374] Subtypes: acetylcholine transmembrane transporter activity [GO:0005277] Sources: GOC:TermGenie Definition: Enables the transfer of an acetate ester from one side of a membrane to the other.